{
  "term_id": "GO:0005811",
  "gene_symbol": "PNPLA3",
  "gene_name": "1-acylglycerol-3-phosphate O-acyltransferase PNPLA3",
  "gene": "UniProtKB:Q9NST1",
  "term_label": "lipid droplet"
}